{
  "gene": "UniProtKB:Q02318",
  "term_id": "GO:0030343",
  "gene_name": "Sterol 26-hydroxylase, mitochondrial",
  "term_label": "vitamin D3 25-hydroxylase activity",
  "gene_symbol": "CYP27A1"
}